{
  "gene": "UniProtKB:Q9UBM7",
  "term_label": "endoplasmic reticulum membrane",
  "gene_name": "7-dehydrocholesterol reductase",
  "term_id": "GO:0005789",
  "gene_symbol": "DHCR7"
}